host cell nuclear envelope [GO:0044199] (cellular component) Definition: The double lipid bilayer that encloses the host cell nucleus, separating its contents from the cytoplasm. It consists of an inner and outer nuclear membrane, with an intermembrane space (20-40 nm wide, also called the perinuclear space) between them. The envelope is supported by the nuclear lamina and contains nuclear pore complexes, which regulate molecular transport. Sources: GOC:jl, GOC:rynl Relationships: is_a host cell nuclear part [GO:0044094]; is part of host cell endomembrane system [GO:0033645]